{
  "gene": "UniProtKB:O60763",
  "gene_name": "General vesicular transport factor p115",
  "term_label": "ER to Golgi transport vesicle membrane",
  "gene_symbol": "USO1",
  "term_id": "GO:0012507"
}